{
  "term_label": "Unknown biological process",
  "term_id": "UNKNOWN:0002",
  "gene_symbol": "SMIM33",
  "gene": "UniProtKB:A0A1B0GW64",
  "gene_name": "Small integral membrane protein 33"
}